protein retention in Golgi apparatus [GO:0045053] (biological process) Definition: The retention of proteins within the Golgi apparatus. Golgi-localized carbohydrate-modifying enzymes have a short N-terminal domain that faces the cytosol, a single transmembrane alpha helix, and a large C-terminal domain that faces the Golgi lumen and that contains the catalytic site. How the membrane-spanning alpha helix in a Golgi enzyme causes its localization and prevents its movement to the plasma membrane is not known. Sources: ISBN:0716731363 Relationships: is a type of GO:0032507; is part of protein localization to Golgi apparatus [GO:0034067] Also known as: protein-Golgi retention, retention of protein in Golgi, maintenance of protein location in Golgi apparatus